{
  "gene_symbol": "MYO7B",
  "gene": "UniProtKB:Q6PIF6",
  "term_id": "GO:0030048",
  "term_label": "actin filament-based movement",
  "gene_name": "Unconventional myosin-VIIb"
}